{
  "gene_symbol": "SCYGR1",
  "term_label": "Unknown cellular component",
  "gene": "UniProtKB:A0A286YEY9",
  "gene_name": "Small cysteine and glycine repeat-containing protein 1",
  "term_id": "UNKNOWN:0003"
}